{
  "gene": "UniProtKB:Q9Y253",
  "term_id": "GO:0005657",
  "term_label": "replication fork",
  "gene_symbol": "POLH",
  "gene_name": "DNA polymerase eta"
}